{
  "gene": "UniProtKB:Q8TD55",
  "gene_symbol": "PLEKHO2",
  "term_id": "GO:0071888",
  "term_label": "macrophage apoptotic process",
  "gene_name": "Pleckstrin homology domain-containing family O member 2"
}